{
  "term_label": "peptide-O-fucosyltransferase activity",
  "term_id": "GO:0046922",
  "gene": "UniProtKB:Q9H488",
  "gene_name": "GDP-fucose protein O-fucosyltransferase 1",
  "gene_symbol": "POFUT1"
}